{
  "gene_name": "Paired box protein Pax-3",
  "term_label": "RNA polymerase II cis-regulatory region sequence-specific DNA binding",
  "gene_symbol": "PAX3",
  "term_id": "GO:0000978",
  "gene": "UniProtKB:P23760"
}